{
  "gene_symbol": "CHGB",
  "term_label": "Unknown molecular function",
  "gene_name": "Secretogranin-1",
  "gene": "UniProtKB:P05060",
  "term_id": "UNKNOWN:0001"
}